{
  "gene_symbol": "ADGRA1",
  "gene_name": "Adhesion G protein-coupled receptor A1",
  "gene": "UniProtKB:Q86SQ6",
  "term_id": "GO:0005886",
  "term_label": "plasma membrane"
}